{
  "term_id": "GO:0003682",
  "gene_symbol": "NPM1",
  "gene_name": "Nucleophosmin",
  "gene": "UniProtKB:P06748",
  "term_label": "chromatin binding"
}